{
  "gene_symbol": "ILKAP",
  "term_id": "GO:0004722",
  "term_label": "protein serine/threonine phosphatase activity",
  "gene_name": "Integrin-linked kinase-associated serine_threonine phosphatase 2C",
  "gene": "UniProtKB:Q9H0C8"
}